cellular response to diosgenin [GO:1905093] (biological process) Definition: Any process that results in a change in state or activity of a cell (in terms of movement, secretion, enzyme production, gene expression, etc.) as a result of a diosgenin stimulus. References: PMID:25765596 Sources: GOC:BHF, GOC:BHF_miRNA, GOC:TermGenie, GOC:bc, GO_REF:0000071 Relationships: is a type of cellular response to sterol [GO:0036315]; is a type of GO:0097306; is a type of GO:1905092; is a type of GO:1905837